{
  "term_label": "transcription elongation by RNA polymerase II",
  "gene_name": "PCI domain-containing protein 2",
  "term_id": "GO:0006368",
  "gene_symbol": "PCID2",
  "gene": "UniProtKB:Q5JVF3"
}